{
  "gene_name": "CAAX prenyl protease 2",
  "gene": "UniProtKB:Q9Y256",
  "term_id": "GO:0004222",
  "gene_symbol": "RCE1",
  "term_label": "metalloendopeptidase activity"
}